{
  "gene": "UniProtKB:O15357",
  "gene_name": "Phosphatidylinositol 3,4,5-trisphosphate 5-phosphatase 2",
  "gene_symbol": "INPPL1",
  "term_id": "GO:0050776",
  "term_label": "regulation of immune response"
}